{
  "gene": "UniProtKB:Q6UWL6",
  "gene_symbol": "KIRREL2",
  "term_label": "plasma membrane",
  "gene_name": "Kin of IRRE-like protein 2",
  "term_id": "GO:0005886"
}